negative regulation of natural killer cell differentiation [GO:0032824] (biological process) Note: Note that immunologists typically use the word 'development' to refer to cells of B or T cell lineages undergoing the process that GO describes as 'cell differentiation'. Subtypes: GO:0032827 Relationships: is a type of negative regulation of natural killer cell activation [GO:0032815]; is a type of GO:0032823; is a type of negative regulation of lymphocyte differentiation [GO:0045620]; negatively regulates natural killer cell differentiation [GO:0001779] Definition: Any process that stops, prevents, or reduces the frequency, rate or extent of natural killer cell differentiation. Also known as: down regulation of natural killer cell differentiation, down-regulation of natural killer cell differentiation, downregulation of natural killer cell differentiation, negative regulation of NK cell differentiation, inhibition of natural killer cell differentiation, negative regulation of natural killer cell development Sources: GOC:mah